diadenosine triphosphate catabolic process [GO:0015964] (biological process) Definition: The chemical reactions and pathways resulting in the breakdown of diadenosine triphosphate, a derivative of the nucleoside adenosine with three phosphate groups attached. Sources: GOC:ai Relationships: is a type of diadenosine polyphosphate catabolic process [GO:0015961] Also known as: diadenosine triphosphate breakdown, diadenosine triphosphate catabolism, diadenosine triphosphate degradation